{
  "term_label": "Unknown molecular function",
  "gene_name": "Cyclin-dependent kinase 2-associated protein 2",
  "term_id": "UNKNOWN:0001",
  "gene_symbol": "CDK2AP2",
  "gene": "UniProtKB:O75956"
}